{
  "gene_name": "Vascular endothelial growth factor D",
  "term_id": "GO:0060754",
  "gene_symbol": "VEGFD",
  "gene": "UniProtKB:O43915",
  "term_label": "positive regulation of mast cell chemotaxis"
}